{
  "term_label": "N-acylphosphatidylethanolamine metabolic process",
  "term_id": "GO:0070292",
  "gene_symbol": "PLAAT5",
  "gene": "UniProtKB:Q96KN8",
  "gene_name": "Phospholipase A and acyltransferase 5"
}